regulation of hydrogen peroxide biosynthetic process [GO:0010728] (biological process) Subtypes: positive regulation of hydrogen peroxide biosynthetic process [GO:0010729], negative regulation of hydrogen peroxide biosynthetic process [GO:0010730] Also known as: regulation of hydrogen peroxide biosynthesis Definition: Any process that modulates the rate, frequency or extent of hydrogen peroxide biosynthesis. The chemical reactions and pathways resulting in the formation of hydrogen peroxide (H2O2), a potentially harmful byproduct of aerobic cellular respiration which can cause damage to DNA. Sources: GOC:dph, GOC:hjd, GOC:tb Relationships: is a type of regulation of hydrogen peroxide metabolic process [GO:0010310]; is a type of regulation of reactive oxygen species biosynthetic process [GO:1903426]; regulates hydrogen peroxide biosynthetic process [GO:0050665]